{
  "gene_symbol": "PCSK4",
  "term_label": "peptide hormone processing",
  "gene": "UniProtKB:Q6UW60",
  "gene_name": "Proprotein convertase subtilisin_kexin type 4",
  "term_id": "GO:0016486"
}